NAD-cap decapping [GO:0110155] (biological process) Relationships: is a type of RNA decapping [GO:0110154] Definition: Cleavage of the 5'-NAD-cap of an RNA. The NAD-cap is present at the 5'-end of some RNAs in both bacetria and eukaryotes. While it promotes RNA stability in bacteria, it promotes RNA decay in eukaryotes. References: PMID:25533955, PMID:28283058, PMID:31101919 Sources: GOC:sp